ethanolamine catabolic process [GO:0046336] (biological process) Definition: The chemical reactions and pathways resulting in the breakdown of ethanolamine (2-aminoethanol), an important water-soluble base of phospholipid (phosphatidylethanolamine). Also known as: ethanolamine breakdown, ethanolamine catabolism, ethanolamine degradation Relationships: is a type of ethanolamine metabolic process [GO:0006580]; is a type of primary alcohol catabolic process [GO:0034310]; is_a biogenic amine catabolic process [GO:0042402]; is a type of GO:1901161 Sources: GOC:ai